{
  "gene": "UniProtKB:Q3LI61",
  "gene_name": "Keratin-associated protein 20-2",
  "gene_symbol": "KRTAP20-2",
  "term_id": "UNKNOWN:0002",
  "term_label": "Unknown biological process"
}